cobyrinic acid a,c-diamide synthase activity [GO:0042242] (molecular function) References: PMID:2172209 Sources: RHEA:26289 Also known as: cobyrinate a c diamide synthase activity, cobyrinate a c-diamide synthase activity, cobyrinate a,c diamide synthase activity, cobyrinate a,c-diamide synthase activity, CobB Relationships: is a type of carbon-nitrogen ligase activity, with glutamine as amido-N-donor [GO:0016884] Definition: Catalysis of the conversion of cobyrinic acid to cobyrinic acid a,c-diamide via the intermediate formation of cobyrinic acid c-monoamide.